{
  "gene": "UniProtKB:Q96PP9",
  "gene_symbol": "GBP4",
  "term_label": "GTP binding",
  "term_id": "GO:0005525",
  "gene_name": "Guanylate-binding protein 4"
}